3-hydroxymethylcephem carbamoyltransferase activity [GO:0047155] (molecular function) Relationships: is a type of carboxyl- or carbamoyltransferase activity [GO:0016743] Definition: Catalysis of the reaction: a 3-hydroxymethylceph-3-em-4-carboxylate + carbamoyl-phosphate = phosphate + a 3-carbamoyloxymethylcephem. Also known as: 3'-hydroxymethylcephem-O-carbamoyltransferase activity, carbamoyl-phosphate:3-hydroxymethylceph-3-em-4-carboxylate carbamoyltransferase activity Sources: EC:2.1.3.7, MetaCyc:2.1.3.7-RXN